{
  "gene_name": "Biogenesis of lysosome-related organelles complex 1 subunit 4",
  "term_id": "UNKNOWN:0001",
  "term_label": "Unknown molecular function",
  "gene": "UniProtKB:Q9NUP1",
  "gene_symbol": "BLOC1S4"
}